{
  "gene_name": "CWF19-like protein 1",
  "gene_symbol": "CWF19L1",
  "term_label": "mRNA splicing, via spliceosome",
  "gene": "UniProtKB:Q69YN2",
  "term_id": "GO:0000398"
}